{
  "gene_symbol": "PRO2829",
  "gene_name": "Putative uncharacterized protein PRO2829",
  "term_id": "UNKNOWN:0002",
  "gene": "UniProtKB:Q9P1C3",
  "term_label": "Unknown biological process"
}